response to vitamin [GO:0033273] (biological process) Relationships: is a type of response to nutrient [GO:0007584] Definition: Any process that results in a change in state or activity of a cell or an organism (in terms of movement, secretion, enzyme production, gene expression, etc.) as a result of a vitamin stimulus. Sources: GOC:sl Subtypes: GO:0010266, response to vitamin K [GO:0032571], GO:0033189, response to vitamin E [GO:0033197], response to vitamin B2 [GO:0033274], GO:0033280, response to vitamin B3 [GO:0033552], GO:0033590, response to L-ascorbic acid [GO:0033591], GO:0034516, response to folic acid [GO:0051593], response to biotin [GO:0070781], cellular response to vitamin [GO:0071295]